polysaccharide transport [GO:0015774] (biological process) Definition: The directed movement of polysaccharides into, out of or within a cell, or between cells, by means of some agent such as a transporter or pore. A polysaccharide is a polymer of many (typically more than 10) monosaccharide residues linked glycosidically. Subtypes: beta-glucan transport [GO:0015775], capsular polysaccharide transport [GO:0015776], arabinan transmembrane transport [GO:0042899], dextrin transport [GO:0042955] Relationships: is a type of carbohydrate transport [GO:0008643]; is part of polysaccharide localization [GO:0033037] Sources: GOC:ai